DNA synthesis involved in mitotic DNA replication [GO:1904860] (BP) References: PMID:16849602 Sources: GOC:TermGenie, GO_REF:0000060 Relationships: is a type of DNA synthesis involved in DNA replication [GO:0090592]; is a type of mitotic cell cycle process [GO:1903047]; is part of mitotic DNA replication [GO:1902969] Definition: Any DNA biosynthetic process that is involved in mitotic DNA replication. Also known as: DNA anabolism involved in DNA replication involved in S phase involved in mitotic cell cycle, DNA anabolism involved in DNA replication involved in S-phase involved in mitotic cell cycle, DNA anabolism involved in mitotic DNA replication, DNA anabolism involved in mitotic cell cycle DNA replication, DNA anabolism involved in mitotic nuclear cell cycle DNA replication, DNA biosynthesis involved in DNA replication involved in S phase involved in mitotic cell cycle, DNA biosynthesis involved in DNA replication involved in S-phase involved in mitotic cell cycle, DNA biosynthesis involved in mitotic DNA replication, DNA biosynthesis involved in mitotic cell cycle DNA replication, DNA biosynthesis involved in mitotic nuclear cell cycle DNA replication, DNA biosynthetic process involved in DNA replication involved in S phase involved in mitotic cell cycle, DNA biosynthetic process involved in DNA replication involved in S-phase involved in mitotic cell cycle, DNA biosynthetic process involved in mitotic DNA replication, DNA biosynthetic process involved in mitotic cell cycle DNA replication, DNA biosynthetic process involved in mitotic nuclear cell cycle DNA replication, DNA formation involved in DNA replication involved in S phase involved in mitotic cell cycle, DNA formation involved in DNA replication involved in S-phase involved in mitotic cell cycle, DNA formation involved in mitotic DNA replication, DNA formation involved in mitotic cell cycle DNA replication, DNA formation involved in mitotic nuclear cell cycle DNA replication, DNA synthesis involved in DNA replication involved in S phase involved in mitotic cell cycle, DNA synthesis involved in DNA replication involved in S-phase involved in mitotic cell cycle, DNA synthesis involved in mitotic cell cycle DNA replication, DNA synthesis involved in mitotic nuclear cell cycle DNA replication, DNA anabolism involved in DNA replication during S phase involved in mitotic cell cycle, DNA anabolism involved in nuclear cell cycle DNA replication involved in mitotic cell cycle, DNA biosynthesis involved in DNA replication during S phase involved in mitotic cell cycle, DNA biosynthesis involved in nuclear cell cycle DNA replication involved in mitotic cell cycle, DNA biosynthetic process involved in DNA replication during S phase involved in mitotic cell cycle, DNA biosynthetic process involved in nuclear cell cycle DNA replication involved in mitotic cell cycle, DNA formation involved in DNA replication during S phase involved in mitotic cell cycle, DNA formation involved in nuclear cell cycle DNA replication involved in mitotic cell cycle, DNA synthesis involved in DNA replication during S phase involved in mitotic cell cycle, DNA synthesis involved in nuclear cell cycle DNA replication involved in mitotic cell cycle